{
  "term_id": "UNKNOWN:0003",
  "gene_name": "RNA-binding protein 33",
  "gene": "UniProtKB:Q96EV2",
  "gene_symbol": "RBM33",
  "term_label": "Unknown cellular component"
}